response to nicotine [GO:0035094] (biological process) Definition: Any process that results in a change in state or activity of a cell or an organism (in terms of movement, secretion, enzyme production, gene expression, etc.) as a result of a nicotine stimulus. Sources: GOC:bf, GOC:ef, ISBN:0198506732, ISBN:0582227089 Relationships: is a type of response to chemical [GO:0042221] Subtypes: cellular response to nicotine [GO:0071316]